{
  "gene": "UniProtKB:P05154",
  "gene_name": "Plasma serine protease inhibitor",
  "term_label": "extracellular space",
  "gene_symbol": "SERPINA5",
  "term_id": "GO:0005615"
}